{
  "gene": "UniProtKB:P01574",
  "term_label": "type I interferon receptor binding",
  "gene_symbol": "IFNB1",
  "gene_name": "Interferon beta",
  "term_id": "GO:0005132"
}